{
  "gene_name": "Transcription factor E2F7",
  "gene_symbol": "E2F7",
  "term_label": "RNA polymerase II transcription regulator complex",
  "gene": "UniProtKB:Q96AV8",
  "term_id": "GO:0090575"
}